{
  "gene": "UniProtKB:A0A096LP55",
  "term_label": "respiratory chain complex III",
  "gene_name": "Cytochrome b-c1 complex subunit 6-like, mitochondrial",
  "term_id": "GO:0045275",
  "gene_symbol": "UQCRHL"
}